{
  "gene": "UniProtKB:Q16322",
  "term_id": "GO:0071805",
  "gene_name": "Potassium voltage-gated channel subfamily A member 10",
  "term_label": "potassium ion transmembrane transport",
  "gene_symbol": "KCNA10"
}